{
  "term_id": "GO:0000981",
  "gene_name": "Zinc finger protein 69",
  "gene": "UniProtKB:Q9UC07",
  "term_label": "DNA-binding transcription factor activity, RNA polymerase II-specific",
  "gene_symbol": "ZNF69"
}